{
  "gene_name": "Ras-related protein Rab-5A",
  "gene": "UniProtKB:P20339",
  "term_label": "dendrite",
  "gene_symbol": "RAB5A",
  "term_id": "GO:0030425"
}